{
  "gene_symbol": "STX7",
  "gene": "UniProtKB:O15400",
  "gene_name": "Syntaxin-7",
  "term_label": "endomembrane system",
  "term_id": "GO:0012505"
}